{
  "term_label": "regulation of inflammatory response",
  "term_id": "GO:0050727",
  "gene": "UniProtKB:Q86W25",
  "gene_name": "NACHT, LRR and PYD domains-containing protein 13",
  "gene_symbol": "NLRP13"
}